{
  "gene_name": "Rap1 GTPase-activating protein 2",
  "term_label": "Unknown biological process",
  "gene": "UniProtKB:Q684P5",
  "term_id": "UNKNOWN:0002",
  "gene_symbol": "RAP1GAP2"
}